{
  "term_label": "hormone activity",
  "term_id": "GO:0005179",
  "gene_symbol": "EPO",
  "gene_name": "Erythropoietin",
  "gene": "UniProtKB:P01588"
}